negative regulation of long-term synaptic depression [GO:1900453] (biological process) Sources: GOC:BHF, GOC:TermGenie Also known as: down regulation of long term depression, down-regulation of long term depression, downregulation of long term depression, inhibition of long term depression, negative regulation of long term depression, down regulation of long term synaptic depression, down-regulation of long term synaptic depression, downregulation of long term synaptic depression, inhibition of long term synaptic depression, down regulation of LTD, down-regulation of LTD, downregulation of LTD, inhibition of LTD, negative regulation of LTD, negative regulation of long term synaptic depression Definition: Any process that stops, prevents or reduces the frequency, rate or extent of long term synaptic depression. Relationships: is a type of negative regulation of biological process [GO:0048519]; is a type of positive regulation of synaptic transmission [GO:0050806]; is a type of regulation of long-term synaptic depression [GO:1900452]; negatively regulates long-term synaptic depression [GO:0060292]